amyloplast [GO:0009501] (cellular component) Relationships: is a type of plastid [GO:0009536] Definition: A plastid whose main function is to synthesize and store starch. Sources: ISBN:0140514031